{
  "term_id": "GO:0032790",
  "gene_symbol": "PELO",
  "gene": "UniProtKB:Q9BRX2",
  "gene_name": "Protein pelota homolog",
  "term_label": "ribosome disassembly"
}